intracellular cAMP-activated cation channel activity involved in regulation of presynaptic membrane potential [GO:0140232] (molecular function) References: PMID:21358644 Definition: Enables the transmembrane transfer of a cation by a channel that opens when intracellular cAMP has been bound by the channel complex or one of its constituent parts, to regulate the presynaptic membrane potential. Also known as: intracellular cAMP activated cation channel activity involved in regulation of presynaptic membrane potential Relationships: is a type of intracellularly cAMP-activated cation channel activity [GO:0005222]; BFO_0000050 regulation of postsynaptic membrane potential [GO:0060078] Note: Note that this term was created for the SynGO project, and will be obsoleted when the SynGO annotations are made in Noctua.